{
  "gene_name": "C-type lectin domain family 2 member A",
  "gene_symbol": "CLEC2A",
  "gene": "UniProtKB:Q6UVW9",
  "term_id": "GO:0048018",
  "term_label": "receptor ligand activity"
}